{
  "term_id": "GO:0005737",
  "gene_name": "Tripartite motif-containing protein 72",
  "term_label": "cytoplasm",
  "gene": "UniProtKB:Q6ZMU5",
  "gene_symbol": "TRIM72"
}